{
  "term_id": "GO:0038023",
  "term_label": "signaling receptor activity",
  "gene": "UniProtKB:Q7Z6A9",
  "gene_name": "B- and T-lymphocyte attenuator",
  "gene_symbol": "BTLA"
}